{
  "term_label": "aspartate transmembrane transport",
  "gene": "UniProtKB:Q9H936",
  "term_id": "GO:0015810",
  "gene_name": "Mitochondrial glutamate carrier 1",
  "gene_symbol": "SLC25A22"
}